{
  "term_id": "GO:0006271",
  "gene_symbol": "MCM7",
  "gene_name": "DNA replication licensing factor MCM7",
  "gene": "UniProtKB:P33993",
  "term_label": "DNA strand elongation involved in DNA replication"
}